{
  "term_id": "GO:0005049",
  "gene_symbol": "XPO7",
  "gene_name": "Exportin-7",
  "term_label": "nuclear export signal receptor activity",
  "gene": "UniProtKB:Q9UIA9"
}